{
  "term_label": "Unknown molecular function",
  "gene_name": "F-box and WD repeat domain containing protein 10B",
  "gene_symbol": "FBXW10B",
  "term_id": "UNKNOWN:0001",
  "gene": "UniProtKB:O95170"
}